{
  "gene": "UniProtKB:P63167",
  "term_id": "GO:0044458",
  "gene_name": "Dynein light chain 1, cytoplasmic",
  "term_label": "motile cilium assembly",
  "gene_symbol": "DYNLL1"
}